{
  "gene": "UniProtKB:Q5TCH4",
  "term_id": "UNKNOWN:0003",
  "gene_symbol": "CYP4A22",
  "term_label": "Unknown cellular component",
  "gene_name": "Cytochrome P450 4A22"
}